{
  "gene_symbol": "SEMA3B",
  "term_label": "negative chemotaxis",
  "term_id": "GO:0050919",
  "gene_name": "Semaphorin-3B",
  "gene": "UniProtKB:Q13214"
}